{
  "gene": "UniProtKB:P78382",
  "gene_name": "CMP-sialic acid transporter",
  "term_id": "GO:0000139",
  "gene_symbol": "SLC35A1",
  "term_label": "Golgi membrane"
}